{
  "gene": "UniProtKB:Q8TAC1",
  "gene_symbol": "RFESD",
  "term_label": "Unknown cellular component",
  "gene_name": "Rieske domain-containing protein",
  "term_id": "UNKNOWN:0003"
}